{
  "gene": "UniProtKB:Q9UKA8",
  "gene_name": "Calcipressin-3",
  "gene_symbol": "RCAN3",
  "term_label": "cytoplasm",
  "term_id": "GO:0005737"
}